{
  "term_label": "Unknown biological process",
  "gene": "UniProtKB:A0A1W2PS18",
  "term_id": "UNKNOWN:0002",
  "gene_name": "Transmembrane protein PMIS2",
  "gene_symbol": "PMIS2"
}